{
  "gene_name": "Phospholipase A and acyltransferase 3",
  "gene": "UniProtKB:P53816",
  "term_id": "GO:0008970",
  "gene_symbol": "PLAAT3",
  "term_label": "phospholipase A1 activity"
}